{
  "gene_symbol": "GREM2",
  "term_id": "GO:0036122",
  "term_label": "BMP binding",
  "gene": "UniProtKB:Q9H772",
  "gene_name": "Gremlin-2"
}